{
  "gene_name": "B-cell lymphoma 6 protein",
  "term_id": "GO:0042092",
  "gene": "UniProtKB:P41182",
  "gene_symbol": "BCL6",
  "term_label": "type 2 immune response"
}